{
  "gene_symbol": "RIIAD1",
  "term_id": "UNKNOWN:0001",
  "gene": "UniProtKB:A6NNX1",
  "gene_name": "RIIa domain-containing protein 1",
  "term_label": "Unknown molecular function"
}